{
  "gene_symbol": "CSH2",
  "gene_name": "Chorionic somatomammotropin hormone 2",
  "term_label": "growth factor activity",
  "gene": "UniProtKB:P0DML3",
  "term_id": "GO:0008083"
}